{
  "gene_symbol": "RAB32",
  "term_label": "endomembrane system",
  "gene": "UniProtKB:Q13637",
  "term_id": "GO:0012505",
  "gene_name": "Ras-related protein Rab-32"
}